{
  "gene_symbol": "CSNK1D",
  "gene": "UniProtKB:P48730",
  "term_id": "GO:0051225",
  "term_label": "spindle assembly",
  "gene_name": "Casein kinase I isoform delta"
}